hard palate morphogenesis [GO:1905748] (biological process) Definition: The developmental process by which a hard palate is generated and organized. Also known as: palatum durum morphogenesis Relationships: is a type of anatomical structure morphogenesis [GO:0009653] References: PMID:23419067 Sources: GOC:TermGenie, GO_REF:0000083